behavioral response to nutrient [GO:0051780] (biological process) Relationships: is a type of behavior [GO:0007610]; is part of response to nutrient [GO:0007584] Definition: Any process that results in a change in the behavior of an organism as a result of a nutrient stimulus. Sources: GOC:ai Subtypes: proboscis extension reflex [GO:0007637] Also known as: behavioural response to nutrient